{
  "term_id": "GO:0051481",
  "gene": "UniProtKB:P14416",
  "term_label": "negative regulation of cytosolic calcium ion concentration",
  "gene_symbol": "DRD2",
  "gene_name": "D(2) dopamine receptor"
}